{
  "gene_name": "Serine_threonine-protein kinase 35",
  "term_label": "negative regulation of G2/M transition of mitotic cell cycle",
  "gene_symbol": "STK35",
  "gene": "UniProtKB:Q8TDR2",
  "term_id": "GO:0010972"
}